response to carbendazim [GO:1901597] (biological process) Relationships: is a type of response to nitrogen compound [GO:1901698]; is a type of response to oxygen-containing compound [GO:1901700] Definition: Any process that results in a change in state or activity of a cell or an organism (in terms of movement, secretion, enzyme production, gene expression, etc.) as a result of a carbendazim stimulus. Subtypes: cellular response to carbendazim [GO:0072762] Sources: GOC:TermGenie